{
  "term_id": "GO:0007411",
  "gene_symbol": "EFNB2",
  "gene": "UniProtKB:P52799",
  "gene_name": "Ephrin-B2",
  "term_label": "axon guidance"
}